{
  "gene": "UniProtKB:P35240",
  "gene_symbol": "NF2",
  "term_label": "regulation of gliogenesis",
  "gene_name": "Merlin",
  "term_id": "GO:0014013"
}